olfactory lobe development [GO:0021988] (biological process) Relationships: is a type of anatomical structure development [GO:0048856]; is part of GO:0021537 Sources: GOC:cls, GOC:dgh, GOC:dph, GOC:jid, GO_REF:0000021 Definition: The progression of the olfactory lobe over time from its initial formation until its mature state. The olfactory lobe is the area of the brain that process the neural inputs for the sense of smell.